mismatch repair involved in maintenance of fidelity involved in DNA-dependent DNA replication [GO:0070716] (biological process) Definition: A mismatch repair process that corrects errors introduced that ensures the accuracy of DNA replication. Relationships: is a type of GO:0006298; is part of DNA-templated DNA replication maintenance of fidelity [GO:0045005] Sources: GOC:BHF, GOC:mah Subtypes: GO:1990516 Also known as: mismatch repair involved in maintenance of fidelity during DNA-dependent DNA replication